{
  "term_id": "GO:0006612",
  "gene_symbol": "RTP4",
  "term_label": "protein targeting to membrane",
  "gene_name": "Receptor-transporting protein 4",
  "gene": "UniProtKB:Q96DX8"
}